{
  "term_label": "chromatin binding",
  "gene_name": "Menin",
  "gene_symbol": "MEN1",
  "gene": "UniProtKB:O00255",
  "term_id": "GO:0003682"
}